{
  "gene": "UniProtKB:P42263",
  "term_label": "AMPA glutamate receptor activity",
  "term_id": "GO:0004971",
  "gene_name": "Glutamate receptor 3",
  "gene_symbol": "GRIA3"
}